{
  "gene": "UniProtKB:Q13227",
  "term_label": "transcription coregulator activity",
  "term_id": "GO:0003712",
  "gene_symbol": "GPS2",
  "gene_name": "G protein pathway suppressor 2"
}